{
  "term_label": "neuronal cell body",
  "gene_name": "Voltage-dependent P_Q-type calcium channel subunit alpha-1A",
  "gene": "UniProtKB:O00555",
  "gene_symbol": "CACNA1A",
  "term_id": "GO:0043025"
}